somatic diversification of immune receptors via germline recombination within a single locus [GO:0002562] (biological process) Subtypes: somatic recombination of T cell receptor gene segments [GO:0002681], somatic recombination of immunoglobulin gene segments [GO:0016447], V(D)J recombination [GO:0033151] Relationships: is a type of somatic diversification of immune receptors [GO:0002200]; is a type of GO:0016444 Definition: The process in which immune receptor genes are diversified through recombination of the germline genetic elements within a single genetic locus. References: PMID:16102575, PMID:16166509 Sources: GOC:add, ISBN:0781735149